{
  "term_id": "GO:0007409",
  "term_label": "axonogenesis",
  "gene_name": "Tripartite motif-containing protein 46",
  "gene": "UniProtKB:Q7Z4K8",
  "gene_symbol": "TRIM46"
}